regulation of DNA-templated transcription elongation [GO:0032784] (biological process) Definition: Any process that modulates the frequency, rate or extent of transcription elongation, the extension of an RNA molecule after transcription initiation and promoter clearance by the addition of ribonucleotides catalyzed by a DNA-dependent RNA polymerase. Relationships: is a type of GO:0006355; regulates DNA-templated transcription elongation [GO:0006354] Also known as: regulation of RNA elongation, regulation of transcriptional elongation, regulation of DNA-dependent transcription, elongation, regulation of DNA-templated transcription, elongation, regulation of transcription elongation, DNA-dependent, transcription elongation regulator activity Sources: GOC:mah, GOC:txnOH Subtypes: negative regulation of DNA-templated transcription, elongation [GO:0032785], GO:0032786, regulation of transcription elongation by RNA polymerase II [GO:0034243], GO:2001207